{
  "gene_symbol": "BNIP3L",
  "gene_name": "BCL2_adenovirus E1B 19 kDa protein-interacting protein 3-like",
  "gene": "UniProtKB:O60238",
  "term_id": "GO:0005741",
  "term_label": "mitochondrial outer membrane"
}